{
  "gene": "UniProtKB:P40616",
  "term_id": "GO:0005737",
  "gene_symbol": "ARL1",
  "gene_name": "ADP-ribosylation factor-like protein 1",
  "term_label": "cytoplasm"
}